{
  "term_label": "defense response to Gram-positive bacterium",
  "gene_name": "Guanylate-binding protein 6",
  "gene_symbol": "GBP6",
  "gene": "UniProtKB:Q6ZN66",
  "term_id": "GO:0050830"
}